positive regulation of acetate catabolic process [GO:0045754] (biological process) Relationships: is a type of positive regulation of catabolic process [GO:0009896]; is a type of regulation of acetate catabolic process [GO:0045734]; is_a positive regulation of small molecule metabolic process [GO:0062013]; positively regulates acetate catabolic process [GO:0045733] Sources: GOC:go_curators Definition: Any process that activates or increases the frequency, rate or extent of the chemical reactions and pathways resulting in the breakdown of acetate. Also known as: positive regulation of acetate breakdown, positive regulation of acetate catabolism, positive regulation of acetate degradation, up regulation of acetate catabolic process, up-regulation of acetate catabolic process, upregulation of acetate catabolic process, activation of acetate catabolic process, stimulation of acetate catabolic process